{
  "gene_name": "Nuclear receptor subfamily 0 group B member 1",
  "term_id": "GO:0007530",
  "term_label": "sex determination",
  "gene_symbol": "NR0B1",
  "gene": "UniProtKB:P51843"
}